regulation of xenophagy [GO:1904415] (BP) Note: An example of this is mouse Tbk1 (UniProt symbol, Q9WUN2) in PMID:21617041 (inferred from mutant phenotype). References: PMID:21617041 Sources: GOC:PARL, GOC:TermGenie, GOC:pad, GO_REF:0000058 Subtypes: negative regulation of xenophagy [GO:1904416], GO:1904417 Relationships: is_a regulation of response to biotic stimulus [GO:0002831]; is a type of regulation of macroautophagy [GO:0016241]; is a type of regulation of response to external stimulus [GO:0032101]; regulates xenophagy [GO:0098792] Definition: Any process that modulates the frequency, rate or extent of xenophagy.